{
  "gene_symbol": "ARID1B",
  "gene": "UniProtKB:Q8NFD5",
  "term_label": "positive regulation of DNA-templated transcription",
  "gene_name": "AT-rich interactive domain-containing protein 1B",
  "term_id": "GO:0045893"
}